PKM2 pyruvate kinase complex [GO:1990361] (cellular component) Note: An example of this is PKM2 in human (P14618) in PMID:24606918 (inferred from direct assay). References: PMID:24606918 Sources: GOC:bhm Definition: A protein complex capable of pyruvate kinase activity. PKM2 only exists as homotetramer when bound to beta-d-fructofuranose 1,6-bisphosphate (CHEBI:28013). Relationships: is a type of pyruvate kinase complex [GO:1902912] Also known as: PKM2 homotetramer